{
  "term_label": "structural constituent of postsynaptic actin cytoskeleton",
  "gene_name": "POTE ankyrin domain family member J",
  "gene_symbol": "POTEJ",
  "term_id": "GO:0098973",
  "gene": "UniProtKB:P0CG39"
}